positive regulation of butyryl-CoA catabolic process to butyrate [GO:1900502] (biological process) Relationships: is a type of positive regulation of amide metabolic process [GO:0034250]; is a type of GO:0045723; is a type of GO:0045937; is_a positive regulation of lipid catabolic process [GO:0050996]; is_a regulation of butyryl-CoA catabolic process to butyrate [GO:1900500]; positively regulates butyryl-CoA catabolic process to butyrate [GO:0044581] Also known as: activation of butyryl-CoA catabolism to butyrate, positive regulation of butyryl-CoA catabolism to butyrate, up regulation of butyryl-CoA catabolic process to butyrate, up regulation of butyryl-CoA catabolism to butyrate, up-regulation of butyryl-CoA catabolic process to butyrate, up-regulation of butyryl-CoA catabolism to butyrate, upregulation of butyryl-CoA catabolic process to butyrate, upregulation of butyryl-CoA catabolism to butyrate, activation of butyryl-CoA catabolic process to butyrate Sources: GOC:TermGenie, GOC:mengo_curators Definition: Any process that activates or increases the frequency, rate or extent of butyryl-CoA catabolic process to butyrate.